{
  "term_label": "neuropeptide binding",
  "gene_symbol": "OPRM1",
  "gene": "UniProtKB:P35372",
  "term_id": "GO:0042923",
  "gene_name": "Mu-type opioid receptor"
}